{
  "gene_symbol": "NPHS2",
  "gene": "UniProtKB:Q9NP85",
  "term_id": "UNKNOWN:0002",
  "gene_name": "Podocin",
  "term_label": "Unknown biological process"
}